regulation of cilium-dependent cell motility [GO:1902019] (biological process) Definition: Any process that modulates the frequency, rate or extent of cilium-dependent cell motility. Sources: GOC:TermGenie, GOC:cilia, GOC:jl Also known as: regulation of cilium cell motility, regulation of ciliary cell motility Relationships: is a type of regulation of cell motility [GO:2000145]; regulates GO:0060285 Subtypes: GO:0060295, negative regulation of cilium-dependent cell motility [GO:1902020], positive regulation of cilium-dependent cell motility [GO:2000155]